{
  "gene_name": "Leucine-rich repeat-containing protein 3C",
  "gene": "UniProtKB:A6NJW4",
  "term_label": "Unknown biological process",
  "term_id": "UNKNOWN:0002",
  "gene_symbol": "LRRC3C"
}